sulfathiazole transmembrane transporter activity [GO:0015546] (MF) Also known as: sulphathiazole transporter activity, bicyclomycin/sulfathiazole:hydrogen antiporter activity Relationships: is a type of amide transmembrane transporter activity [GO:0042887]; is a type of azole transmembrane transporter activity [GO:1901474]; is a type of sulfur compound transmembrane transporter activity [GO:1901682]; is part of sulfathiazole transmembrane transport [GO:1902599] Definition: Enables the transfer of sulfathiazole from one side of a membrane to the other. Sulfathiazole is an antibacterial agent of the sulfonamide group. Sources: GOC:curators